{
  "gene": "UniProtKB:Q16763",
  "term_label": "nucleus",
  "gene_symbol": "UBE2S",
  "term_id": "GO:0005634",
  "gene_name": "Ubiquitin-conjugating enzyme E2 S"
}